{
  "gene_name": "Pyruvate kinase PKM",
  "term_label": "cellular response to insulin stimulus",
  "gene": "UniProtKB:P14618",
  "term_id": "GO:0032869",
  "gene_symbol": "PKM"
}